{
  "gene_name": "Glucocorticoid-induced transcript 1 protein",
  "gene": "UniProtKB:Q86VQ1",
  "term_label": "cytoplasm",
  "term_id": "GO:0005737",
  "gene_symbol": "GLCCI1"
}